{
  "term_id": "UNKNOWN:0003",
  "gene_name": "Protein KRBA1",
  "gene": "UniProtKB:A5PL33",
  "gene_symbol": "KRBA1",
  "term_label": "Unknown cellular component"
}